CAF-1 complex [GO:0033186] (cellular component) Definition: A conserved heterotrimeric protein complex that promotes histone H3 and H4 deposition onto newly synthesized DNA during replication or DNA repair; specifically facilitates replication-dependent nucleosome assembly with the major histone H3 (H3.1). In many species the CAF-1 subunits are designated p150, p60, and p48. Relationships: is a type of GO:0032991 Also known as: chromatin assembly factor 1 complex Note: In yeast the subunits are MSI1/p50, CAC2/p60 and CAC1/p90. References: PMID:17065558, PMID:17083276